{
  "gene_symbol": "LIN7A",
  "gene_name": "Protein lin-7 homolog A",
  "term_id": "GO:0097025",
  "term_label": "MPP7-DLG1-LIN7 complex",
  "gene": "UniProtKB:O14910"
}